{
  "term_label": "regulation of synaptic transmission, glutamatergic",
  "gene": "UniProtKB:O15303",
  "gene_name": "Metabotropic glutamate receptor 6",
  "term_id": "GO:0051966",
  "gene_symbol": "GRM6"
}